negative regulation of humoral immune response [GO:0002921] (biological process) Definition: Any process that stops, prevents, or reduces the frequency, rate, or extent of a humoral immune response. Relationships: is a type of regulation of humoral immune response [GO:0002920]; is a type of negative regulation of immune response [GO:0050777]; negatively regulates humoral immune response [GO:0006959] Subtypes: negative regulation of humoral immune response mediated by circulating immunoglobulin [GO:0002924], GO:0008348, negative regulation of complement activation [GO:0045916] Sources: GOC:add Also known as: down regulation of humoral immune response, down-regulation of humoral immune response, downregulation of humoral immune response, inhibition of humoral immune response